{
  "gene_name": "Fatty acid-binding protein, liver",
  "term_label": "fatty acid transport",
  "gene": "UniProtKB:P07148",
  "gene_symbol": "FABP1",
  "term_id": "GO:0015908"
}